intestinal iron absorption [GO:0160179] (biological process) References: PMID:16054062, PMID:17729393 Definition: A process in which iron is taken up from the contents of the intestine. Relationships: is a type of intestinal absorption [GO:0050892]